negative regulation of translational fidelity [GO:0045902] (biological process) Definition: Any process that decreases the ability of the translational apparatus to interpret the genetic code. Also known as: down regulation of translational fidelity, down-regulation of translational fidelity, downregulation of translational fidelity, inhibition of translational fidelity Sources: GOC:dph, GOC:tb Relationships: is_a regulation of translational fidelity [GO:0006450]; is a type of GO:0017148